{
  "gene": "UniProtKB:Q01650",
  "term_id": "GO:0003333",
  "gene_name": "Large neutral amino acids transporter small subunit 1",
  "gene_symbol": "SLC7A5",
  "term_label": "amino acid transmembrane transport"
}